myoblast fusion [GO:0007520] (biological process) Relationships: is a type of GO:0000768; is part of myotube differentiation [GO:0014902] Regulation: RO_0002211 by regulation of myoblast fusion [GO:1901739]; negatively regulated by negative regulation of myoblast fusion [GO:1901740]; positively regulated by GO:1901741 Definition: A process in which non-proliferating myoblasts fuse to existing fibers or to myotubes to form new fibers. A myoblast is a mononucleate cell type that, by fusion with other myoblasts, gives rise to the myotubes that eventually develop into skeletal muscle fibers. Sources: CL:0000056, GOC:mtg_muscle Subtypes: myoblast fusion involved in skeletal muscle regeneration [GO:0014905]